{
  "gene": "UniProtKB:Q7Z7M9",
  "term_id": "GO:0005794",
  "gene_symbol": "GALNT5",
  "gene_name": "Polypeptide N-acetylgalactosaminyltransferase 5",
  "term_label": "Golgi apparatus"
}